sesquithujene synthase activity [GO:0102304] (molecular function) Relationships: is a type of carbon-oxygen lyase activity, acting on phosphates [GO:0016838] Definition: Catalysis of the reaction: 2-trans,6-trans-farnesyl diphosphate(3-) = 7-epi-sesquithujene + diphosphoric acid. Sources: EC:4.2.3.102, GOC:pz